{
  "gene_name": "Myocardin",
  "gene": "UniProtKB:Q8IZQ8",
  "term_label": "transcription coactivator activity",
  "gene_symbol": "MYOCD",
  "term_id": "GO:0003713"
}